{
  "gene_symbol": "IGFBP1",
  "term_label": "extracellular space",
  "term_id": "GO:0005615",
  "gene_name": "Insulin-like growth factor-binding protein 1",
  "gene": "UniProtKB:P08833"
}